{
  "gene_name": "Golgin subfamily A member 6-like protein 25",
  "term_id": "UNKNOWN:0001",
  "gene": "UniProtKB:P0DX01",
  "gene_symbol": "GOLGA6L25",
  "term_label": "Unknown molecular function"
}